{
  "gene_symbol": "DTNA",
  "term_id": "UNKNOWN:0001",
  "gene": "UniProtKB:Q9Y4J8",
  "gene_name": "Dystrobrevin alpha",
  "term_label": "Unknown molecular function"
}